{
  "term_id": "GO:0032590",
  "term_label": "dendrite membrane",
  "gene_name": "Gamma-aminobutyric acid receptor subunit alpha-6",
  "gene": "UniProtKB:Q16445",
  "gene_symbol": "GABRA6"
}